{
  "term_id": "GO:0016485",
  "gene_symbol": "PRSS50",
  "gene": "UniProtKB:Q9UI38",
  "term_label": "protein processing",
  "gene_name": "Probable threonine protease PRSS50"
}